{
  "term_label": "oxalate transmembrane transporter activity",
  "gene_symbol": "SLC26A4",
  "term_id": "GO:0019531",
  "gene": "UniProtKB:O43511",
  "gene_name": "Pendrin"
}